carbazole catabolic process [GO:0046232] (biological process) Also known as: carbazole breakdown, carbazole catabolism, carbazole degradation Sources: GOC:ai Relationships: is a type of GO:0042178 Definition: The chemical reactions and pathways resulting in the breakdown of carbazole, a heterocyclic aromatic compound containing a dibenzopyrrole system that is produced during coal gasification and is present in cigarette smoke. Coal tar produced at high temperature contains an average of 1.5% carbazole. It is used widely in synthesis of dyes, pharmaceuticals, and plastics and is a suspected carcinogen.